{
  "gene_name": "UDP-glucuronosyltransferase 3A1",
  "term_id": "UNKNOWN:0002",
  "gene_symbol": "UGT3A1",
  "term_label": "Unknown biological process",
  "gene": "UniProtKB:Q6NUS8"
}